{
  "term_id": "GO:0043161",
  "term_label": "proteasome-mediated ubiquitin-dependent protein catabolic process",
  "gene": "UniProtKB:Q8WU17",
  "gene_name": "E3 ubiquitin-protein ligase RNF139",
  "gene_symbol": "RNF139"
}